positive regulation of vascular endothelial growth factor receptor signaling pathway [GO:0030949] (biological process) Also known as: positive regulation of VEGF receptor signaling pathway, positive regulation of VEGF receptor signalling pathway, positive regulation of vascular endothelial growth factor receptor signalling pathway, up regulation of vascular endothelial growth factor receptor signaling pathway, up-regulation of vascular endothelial growth factor receptor signaling pathway, upregulation of vascular endothelial growth factor receptor signaling pathway, activation of vascular endothelial growth factor receptor signaling pathway, stimulation of vascular endothelial growth factor receptor signaling pathway Sources: GOC:dgh Definition: Any process that activates or increases the frequency, rate or extent of vascular endothelial growth factor receptor signaling pathway activity. Relationships: is a type of positive regulation of signal transduction [GO:0009967]; is a type of regulation of vascular endothelial growth factor receptor signaling pathway [GO:0030947]; positively regulates vascular endothelial growth factor receptor signaling pathway [GO:0048010]